{
  "gene_name": "HAUS augmin-like complex subunit 1",
  "gene": "UniProtKB:Q96CS2",
  "gene_symbol": "HAUS1",
  "term_label": "centrosome cycle",
  "term_id": "GO:0007098"
}